{
  "gene": "UniProtKB:P28288",
  "term_id": "GO:0006635",
  "gene_symbol": "ABCD3",
  "term_label": "fatty acid beta-oxidation",
  "gene_name": "ATP-binding cassette sub-family D member 3"
}